{
  "gene": "UniProtKB:P49789",
  "gene_symbol": "FHIT",
  "gene_name": "Bis(5'-adenosyl)-triphosphatase",
  "term_label": "purine nucleotide metabolic process",
  "term_id": "GO:0006163"
}